{
  "term_label": "Unknown molecular function",
  "gene_name": "Small integral membrane protein 12",
  "term_id": "UNKNOWN:0001",
  "gene_symbol": "SMIM12",
  "gene": "UniProtKB:Q96EX1"
}